{
  "term_id": "GO:0007029",
  "gene": "UniProtKB:Q8NHH9",
  "gene_name": "Atlastin-2",
  "term_label": "endoplasmic reticulum organization",
  "gene_symbol": "ATL2"
}